{
  "gene": "UniProtKB:Q96Q89",
  "gene_name": "Kinesin-like protein KIF20B",
  "gene_symbol": "KIF20B",
  "term_label": "microtubule motor activity",
  "term_id": "GO:0003777"
}